{
  "gene_symbol": "PDCD1LG2",
  "gene": "UniProtKB:Q9BQ51",
  "term_label": "negative regulation of T cell proliferation",
  "term_id": "GO:0042130",
  "gene_name": "Programmed cell death 1 ligand 2"
}